central nervous system neuron differentiation [GO:0021953] (biological process) Relationships: is a type of neuron differentiation [GO:0030182]; is part of central nervous system development [GO:0007417] Subtypes: ventral spinal cord interneuron differentiation [GO:0021514], spinal cord motor neuron differentiation [GO:0021522], spinal cord association neuron differentiation [GO:0021527], commissural neuron differentiation in spinal cord [GO:0021528], GO:0021701, cerebellar Purkinje cell differentiation [GO:0021702], cerebellar granule cell differentiation [GO:0021707], Lugaro cell differentiation [GO:0021708], GO:0021709, GO:0021710, cerebellar unipolar brush cell differentiation [GO:0021711], candelabrum cell differentiation [GO:0021712], GO:0021755, pyramidal neuron differentiation [GO:0021859], forebrain neuron differentiation [GO:0021879], amacrine cell differentiation [GO:0035881], retrotrapezoid nucleus neuron differentiation [GO:0061452], midbrain dopaminergic neuron differentiation [GO:1904948], GO:1905275 Sources: GOC:cls, GOC:dgh, GOC:dph, GOC:jid, GO_REF:0000021 Definition: The process in which a relatively unspecialized cell acquires specialized features of a neuron whose cell body resides in the central nervous system.